{
  "term_label": "Unknown molecular function",
  "gene": "UniProtKB:Q9NWN3",
  "term_id": "UNKNOWN:0001",
  "gene_name": "F-box only protein 34",
  "gene_symbol": "FBXO34"
}